{
  "gene_name": "Epididymal-specific lipocalin-6",
  "term_id": "UNKNOWN:0001",
  "gene_symbol": "LCN6",
  "gene": "UniProtKB:P62502",
  "term_label": "Unknown molecular function"
}